{
  "term_label": "immunoglobulin complex",
  "gene_name": "Immunoglobulin lambda variable 3-1",
  "gene": "UniProtKB:P01715",
  "term_id": "GO:0019814",
  "gene_symbol": "IGLV3-1"
}